{
  "gene_symbol": "PANX3",
  "term_label": "wide pore channel activity",
  "gene_name": "Pannexin-3",
  "term_id": "GO:0022829",
  "gene": "UniProtKB:Q96QZ0"
}